{
  "term_id": "GO:0043161",
  "gene": "UniProtKB:Q6PJ21",
  "gene_name": "SPRY domain-containing SOCS box protein 3",
  "gene_symbol": "SPSB3",
  "term_label": "proteasome-mediated ubiquitin-dependent protein catabolic process"
}